{
  "term_label": "protein sumoylation",
  "term_id": "GO:0016925",
  "gene_symbol": "CBX4",
  "gene_name": "E3 SUMO-protein ligase CBX4",
  "gene": "UniProtKB:O00257"
}